response to platelet-derived growth factor [GO:0036119] (biological process) Relationships: is_a response to growth factor [GO:0070848] Also known as: response to PDGF stimulus, response to platelet-derived growth factor stimulus Sources: GOC:yaf Subtypes: cellular response to platelet-derived growth factor stimulus [GO:0036120] Definition: Any process that results in a change in state or activity of a cell or an organism (in terms of movement, secretion, enzyme production, gene expression, etc.) as a result of a platelet-derived growth factor stimulus.